negative regulation of skeletal muscle cell proliferation [GO:0014859] (biological process) Definition: Any process that stops, prevents, or reduces the frequency, rate or extent of skeletal muscle cell proliferation. Relationships: is a type of negative regulation of cell population proliferation [GO:0008285]; is_a regulation of skeletal muscle cell proliferation [GO:0014857]; negatively regulates skeletal muscle cell proliferation [GO:0014856] Subtypes: GO:1902723 Sources: CL:0000188, GOC:ef, GOC:mtg_muscle